{
  "gene_name": "Myelin regulatory factor",
  "gene_symbol": "MYRF",
  "gene": "UniProtKB:Q9Y2G1",
  "term_label": "nucleus",
  "term_id": "GO:0005634"
}